{
  "term_id": "GO:0010510",
  "gene_symbol": "PDK2",
  "gene": "UniProtKB:Q15119",
  "term_label": "regulation of pyruvate decarboxylation to acetyl-CoA",
  "gene_name": "[Pyruvate dehydrogenase (acetyl-transferring)] kinase isozyme 2, mitochondrial"
}